{
  "gene": "UniProtKB:P26641",
  "gene_name": "Elongation factor 1-gamma",
  "term_id": "GO:0005634",
  "term_label": "nucleus",
  "gene_symbol": "EEF1G"
}